alcohol dehydrogenase (NAD+) activity [GO:0004022] (molecular function) Relationships: is a type of alcohol dehydrogenase [NAD(P)+] activity [GO:0018455] Also known as: alcohol dehydrogenase activity, primary alcohol dehydrogenase, aldo-keto reductase (NAD) activity, aldehyde dehydrogenase (NAD) activity, aliphatic alcohol dehydrogenase, ethanol dehydrogenase, yeast alcohol dehydrogenase, ADH, NAD-dependent alcohol dehydrogenase, NAD-specific aromatic alcohol dehydrogenase, NADH-alcohol dehydrogenase, NADH-aldehyde dehydrogenase, alcohol:NAD+ oxidoreductase Subtypes: L-iditol 2-dehydrogenase (NAD+) activity [GO:0003939], octanol dehydrogenase (NAD+) activity [GO:0004552], all-trans-retinol dehydrogenase (NAD+) activity [GO:0004745], xanthoxin dehydrogenase (NAD+) activity [GO:0010301], aryl-alcohol dehydrogenase (NAD+) activity [GO:0018456], perillyl-alcohol dehydrogenase (NAD+) activity [GO:0018457], indole-3-acetaldehyde reductase (NADH) activity [GO:0047018], hexadecanol dehydrogenase (NAD+) activity [GO:0047978], methanol dehydrogenase (NAD+) activity [GO:0050093], inositol 2-dehydrogenase (NAD+) activity [GO:0050112], 3-methylbutanal reductase (NADH) activity [GO:0052676], 11-cis-retinol dehydrogenase (NAD+) activity [GO:0106429], ethanol dehydrogenase (NAD+) activity [GO:0120542], butanol dehydrogenase (NAD+) activity [GO:1990362] Definition: Catalysis of the reaction: an alcohol + NAD+ = an aldehyde or ketone + NADH + H+. Sources: EC:1.1.1.1